{
  "gene_symbol": "SHANK2",
  "gene_name": "SH3 and multiple ankyrin repeat domains protein 2",
  "term_label": "ionotropic glutamate receptor binding",
  "gene": "UniProtKB:Q9UPX8",
  "term_id": "GO:0035255"
}